{
  "term_label": "protein-macromolecule adaptor activity",
  "gene_name": "Vinexin",
  "term_id": "GO:0030674",
  "gene_symbol": "SORBS3",
  "gene": "UniProtKB:O60504"
}